snRNA processing [GO:0016180] (biological process) References: PMID:15196465, PMID:31815536 Definition: Any process involved in the conversion of a primary small nuclear RNA (snRNA) transcript into a mature snRNA molecule. The primary function of snRNAs is processing pre-messenger RNA in the nucleus. They have also been shown to aid in the regulation of transcription factors (7SK RNA) or RNA polymerase II (B2 RNA), and maintaining the telomeres. Subtypes: snRNA 3'-end processing [GO:0034472], GO:0040031, GO:1990273 Relationships: is a type of GO:0006396; is a type of snRNA metabolic process [GO:0016073] Also known as: snRNA maturation, snRNA production